{
  "gene_name": "Raftlin-2",
  "term_id": "UNKNOWN:0001",
  "gene_symbol": "RFTN2",
  "gene": "UniProtKB:Q52LD8",
  "term_label": "Unknown molecular function"
}